{
  "term_id": "GO:0008395",
  "gene_name": "Cytochrome P450 2U1",
  "gene": "UniProtKB:Q7Z449",
  "term_label": "steroid hydroxylase activity",
  "gene_symbol": "CYP2U1"
}